{
  "gene_name": "Immunoglobulin kappa variable 1-6",
  "gene_symbol": "IGKV1-6",
  "term_id": "UNKNOWN:0001",
  "gene": "UniProtKB:A0A0C4DH72",
  "term_label": "Unknown molecular function"
}